{
  "gene": "UniProtKB:Q9NR56",
  "term_label": "nucleoplasm",
  "gene_symbol": "MBNL1",
  "term_id": "GO:0005654",
  "gene_name": "Muscleblind-like protein 1"
}